{
  "term_label": "Unknown biological process",
  "gene_name": "Heparan sulfate glucosamine 3-O-sulfotransferase 5",
  "gene_symbol": "HS3ST5",
  "gene": "UniProtKB:Q8IZT8",
  "term_id": "UNKNOWN:0002"
}